{
  "term_label": "plasma membrane",
  "gene_name": "Amiloride-sensitive amine oxidase [copper-containing]",
  "gene": "UniProtKB:P19801",
  "term_id": "GO:0005886",
  "gene_symbol": "AOC1"
}